interleukin-17A receptor activity [GO:0038174] (molecular function) Definition: Combining with the cytokine interleukin-17A and transmitting the signal from one side of the membrane to the other to initiate a change in cell activity. Sources: GOC:bf, GOC:jc, GOC:signaling Relationships: is a type of interleukin-17 receptor activity [GO:0030368]; is part of interleukin-17A-mediated signaling pathway [GO:0038173]